{
  "gene_symbol": "UCK1",
  "gene_name": "Uridine-cytidine kinase 1",
  "term_label": "Unknown biological process",
  "gene": "UniProtKB:Q9HA47",
  "term_id": "UNKNOWN:0002"
}